{
  "term_id": "UNKNOWN:0002",
  "term_label": "Unknown biological process",
  "gene": "UniProtKB:Q5HYW3",
  "gene_symbol": "RTL5",
  "gene_name": "Retrotransposon Gag-like protein 5"
}